{
  "gene": "UniProtKB:Q9H1H9",
  "gene_symbol": "KIF13A",
  "term_id": "GO:0006886",
  "gene_name": "Kinesin-like protein KIF13A",
  "term_label": "intracellular protein transport"
}